{
  "gene_symbol": "C7orf50",
  "gene_name": "Uncharacterized protein C7orf50",
  "term_id": "UNKNOWN:0001",
  "term_label": "Unknown molecular function",
  "gene": "UniProtKB:Q9BRJ6"
}